{
  "term_id": "UNKNOWN:0001",
  "gene_symbol": "ORM1",
  "gene_name": "Alpha-1-acid glycoprotein 1",
  "gene": "UniProtKB:P02763",
  "term_label": "Unknown molecular function"
}